{
  "gene_name": "C-C chemokine receptor type 5",
  "gene_symbol": "CCR5",
  "term_label": "cell chemotaxis",
  "gene": "UniProtKB:P51681",
  "term_id": "GO:0060326"
}